{
  "gene": "UniProtKB:P24539",
  "gene_name": "ATP synthase F(0) complex subunit B1, mitochondrial",
  "term_id": "GO:0046933",
  "gene_symbol": "ATP5PB",
  "term_label": "proton-transporting ATP synthase activity, rotational mechanism"
}